{
  "gene": "UniProtKB:Q07352",
  "gene_name": "mRNA decay activator protein ZFP36L1",
  "term_label": "mRNA regulatory element binding translation repressor activity",
  "gene_symbol": "ZFP36L1",
  "term_id": "GO:0000900"
}